{
  "term_id": "UNKNOWN:0001",
  "gene": "UniProtKB:Q9NX01",
  "gene_name": "Thioredoxin-like protein 4B",
  "term_label": "Unknown molecular function",
  "gene_symbol": "TXNL4B"
}